{
  "gene": "UniProtKB:A4D0T7",
  "term_label": "Unknown molecular function",
  "term_id": "UNKNOWN:0001",
  "gene_symbol": "SMIM30",
  "gene_name": "Small integral membrane protein 30"
}